{
  "term_id": "UNKNOWN:0002",
  "gene_name": "Centrosomal protein 43",
  "term_label": "Unknown biological process",
  "gene_symbol": "CEP43",
  "gene": "UniProtKB:O95684"
}